{
  "term_id": "GO:0050911",
  "term_label": "detection of chemical stimulus involved in sensory perception of smell",
  "gene_symbol": "OR2T8",
  "gene_name": "Olfactory receptor 2T8",
  "gene": "UniProtKB:A6NH00"
}